{
  "term_id": "UNKNOWN:0001",
  "term_label": "Unknown molecular function",
  "gene": "UniProtKB:Q8N1G0",
  "gene_name": "Zinc finger protein 687",
  "gene_symbol": "ZNF687"
}